neural plate thickening [GO:0021991] (biological process) Definition: The process of apical-basal elongation of individual ectodermal cells during the formation of the neural placode. References: PMID:15806586 Sources: GOC:cls, GOC:dgh, GOC:dph, GOC:jid, GO_REF:0000021 Relationships: is a type of morphogenesis of an epithelial sheet [GO:0002011]; is a type of embryonic morphogenesis [GO:0048598]; is part of neural plate morphogenesis [GO:0001839]